SCF-Saf1/Pof9 ubiquitin ligase complex [GO:0097668] (cellular component) Relationships: is a type of GO:0019005 References: PMID:11283612, PMID:15147268 Sources: GOC:jd, GOC:vw Definition: An SCF ubiquitin ligase complex in which the F-box protein is Saf1 in S. cerevisiae (Pof9 in S. pombe).